{
  "term_label": "mitochondrial matrix",
  "gene": "UniProtKB:Q9BRT2",
  "gene_symbol": "UQCC2",
  "gene_name": "Ubiquinol-cytochrome-c reductase complex assembly factor 2",
  "term_id": "GO:0005759"
}